{
  "term_label": "immune response-inhibiting cell surface receptor signaling pathway",
  "gene_name": "Leukocyte immunoglobulin-like receptor subfamily B member 3",
  "gene_symbol": "LILRB3",
  "gene": "UniProtKB:O75022",
  "term_id": "GO:0002767"
}